negative regulation of cytoplasmic translation [GO:2000766] (biological process) Definition: Any process that stops, prevents or reduces the frequency, rate or extent of cytoplasmic translation. Sources: GOC:obol Relationships: is a type of negative regulation of translation [GO:0017148]; is a type of regulation of cytoplasmic translation [GO:2000765]; negatively regulates GO:0002181 Subtypes: negative regulation of cytoplasmic translational elongation [GO:1900248]